{
  "gene_name": "Synaptosomal-associated protein 25",
  "gene": "UniProtKB:P60880",
  "term_id": "GO:0031629",
  "gene_symbol": "SNAP25",
  "term_label": "synaptic vesicle fusion to presynaptic active zone membrane"
}